mating projection tip polarisome [GO:0031563] (cellular component) Relationships: is a type of polarisome [GO:0000133]; is part of mating projection tip [GO:0043332] Definition: Protein complex that has a role in determining cell polarity, found at the tip of the mating projection in unicellular fungi exposed to mating pheromone. References: PMID:14734532